{
  "term_label": "Unknown biological process",
  "term_id": "UNKNOWN:0002",
  "gene_name": "Coiled-coil domain-containing protein 138",
  "gene": "UniProtKB:Q96M89",
  "gene_symbol": "CCDC138"
}